{
  "gene_symbol": "CPZ",
  "term_id": "GO:0004181",
  "gene_name": "Carboxypeptidase Z",
  "gene": "UniProtKB:Q66K79",
  "term_label": "metallocarboxypeptidase activity"
}